{
  "term_id": "GO:0090090",
  "gene_symbol": "DKK3",
  "term_label": "negative regulation of canonical Wnt signaling pathway",
  "gene": "UniProtKB:Q9UBP4",
  "gene_name": "Dickkopf-related protein 3"
}